proteasome core complex import into nucleus [GO:1990236] (biological process) Definition: The directed movement of the proteasome core complex (AKA core particle (CP)) from the cytoplasm into the nucleus. References: PMID:23982732 Sources: GOC:dos, GOC:rb Relationships: is a type of import into nucleus [GO:0051170]